response to interleukin-17 [GO:0097396] (biological process) Definition: Any process that results in a change in state or activity of a cell or an organism (in terms of movement, secretion, enzyme production, gene expression, etc.) as a result of an interleukin-17 stimulus. Relationships: is a type of response to cytokine [GO:0034097] Also known as: response to IL-17 Sources: GOC:pr Subtypes: cellular response to interleukin-17 [GO:0097398]